{
  "gene_symbol": "TSPAN7",
  "gene": "UniProtKB:P41732",
  "gene_name": "Tetraspanin-7",
  "term_label": "plasma membrane",
  "term_id": "GO:0005886"
}